{
  "gene": "UniProtKB:P35749",
  "term_label": "actomyosin structure organization",
  "gene_symbol": "MYH11",
  "gene_name": "Myosin-11",
  "term_id": "GO:0031032"
}